{
  "gene_symbol": "OR10A7",
  "term_id": "GO:0050911",
  "gene_name": "Olfactory receptor 10A7",
  "term_label": "detection of chemical stimulus involved in sensory perception of smell",
  "gene": "UniProtKB:Q8NGE5"
}